{
  "gene_name": "Syntaxin-8",
  "gene": "UniProtKB:Q9UNK0",
  "term_id": "GO:0031201",
  "gene_symbol": "STX8",
  "term_label": "SNARE complex"
}